{
  "term_id": "GO:0000981",
  "term_label": "DNA-binding transcription factor activity, RNA polymerase II-specific",
  "gene_name": "Paired box protein Pax-6",
  "gene": "UniProtKB:P26367",
  "gene_symbol": "PAX6"
}